lumenal side of trans-Golgi network transport vesicle membrane [GO:0098540] (cellular component) Also known as: internal side of trans-Golgi network transport vesicle membrane Relationships: is a type of lumenal side of transport vesicle membrane [GO:0098538]; is part of trans-Golgi network transport vesicle membrane [GO:0012510] Sources: GOC:ab Definition: The side (leaflet) of the trans-Golgi network transport vesicle membrane that faces the lumen.